{
  "gene_name": "Aldo-keto reductase family 1 member D1",
  "term_id": "GO:0047086",
  "gene": "UniProtKB:P51857",
  "term_label": "ketosteroid monooxygenase activity",
  "gene_symbol": "AKR1D1"
}